{
  "gene_symbol": "TRAPPC12",
  "gene": "UniProtKB:Q8WVT3",
  "gene_name": "Trafficking protein particle complex subunit 12",
  "term_id": "UNKNOWN:0001",
  "term_label": "Unknown molecular function"
}